{
  "gene_symbol": "OR9Q2",
  "gene_name": "Olfactory receptor 9Q2",
  "gene": "UniProtKB:Q8NGE9",
  "term_id": "GO:0004984",
  "term_label": "olfactory receptor activity"
}